{
  "gene": "UniProtKB:O95777",
  "gene_symbol": "LSM8",
  "gene_name": "U6 snRNA-associated Sm-like protein LSm8",
  "term_label": "mRNA splicing, via spliceosome",
  "term_id": "GO:0000398"
}